ciliary targeting signal binding [GO:1990473] (molecular function) Definition: Binding to a ciliary targeting sequence, a specific peptide sequence that acts as a signal to localize a membrane protein to the ciliary membrane. Also known as: CTS binding Relationships: is a type of GO:0005048 References: PMID:18256283, PMID:19575670, PMID:20603001, PMID:20697559 Sources: GOC:krc